{
  "term_label": "axonogenesis",
  "term_id": "GO:0007409",
  "gene_name": "Dedicator of cytokinesis protein 7",
  "gene": "UniProtKB:Q96N67",
  "gene_symbol": "DOCK7"
}